{
  "gene": "UniProtKB:Q9C0H5",
  "term_id": "UNKNOWN:0002",
  "gene_symbol": "ARHGAP39",
  "term_label": "Unknown biological process",
  "gene_name": "Rho GTPase-activating protein 39"
}